{
  "term_label": "Unknown biological process",
  "gene": "UniProtKB:Q5VU97",
  "gene_symbol": "CACHD1",
  "gene_name": "VWFA and cache domain-containing protein 1",
  "term_id": "UNKNOWN:0002"
}